{
  "term_id": "GO:0007032",
  "gene_name": "Pleckstrin homology domain-containing family J member 1",
  "gene": "UniProtKB:Q9NW61",
  "gene_symbol": "PLEKHJ1",
  "term_label": "endosome organization"
}